{
  "gene_name": "Fibronectin",
  "term_label": "nervous system development",
  "term_id": "GO:0007399",
  "gene": "UniProtKB:P02751",
  "gene_symbol": "FN1"
}